{
  "term_label": "Golgi apparatus",
  "gene_symbol": "ZDHHC14",
  "gene": "UniProtKB:Q8IZN3",
  "term_id": "GO:0005794",
  "gene_name": "Palmitoyltransferase ZDHHC14"
}